{
  "gene_symbol": "VIL1",
  "gene_name": "Villin-1",
  "term_id": "GO:0051016",
  "gene": "UniProtKB:P09327",
  "term_label": "barbed-end actin filament capping"
}